regulation of biomineral tissue development [GO:0070167] (biological process) Subtypes: regulation of bone mineralization [GO:0030500], negative regulation of biomineral tissue development [GO:0070168], GO:0070169, GO:0070170, regulation of shell calcification [GO:1905648] Relationships: is a type of GO:2000026; regulates biomineral tissue development [GO:0031214] Sources: GOC:mah Definition: Any process that modulates the frequency, rate or extent of biomineral tissue development, the formation of hard tissues that consist mainly of inorganic compounds.